microtubule polymerization or depolymerization [GO:0031109] (biological process) Subtypes: microtubule depolymerization [GO:0007019], microtubule polymerization [GO:0046785] Definition: Assembly or disassembly of microtubules by the addition or removal of tubulin heterodimers from a microtubule. Relationships: is a type of GO:0000226 Sources: GOC:mah Regulation: regulated by regulation of microtubule polymerization or depolymerization [GO:0031110]; negatively regulated by negative regulation of microtubule polymerization or depolymerization [GO:0031111]; positively regulated by GO:0031112 Also known as: microtubule dynamics